{
  "term_id": "UNKNOWN:0001",
  "gene": "UniProtKB:Q8NG94",
  "term_label": "Unknown molecular function",
  "gene_name": "Olfactory receptor 11H1",
  "gene_symbol": "OR11H1"
}